{
  "gene": "UniProtKB:Q9NXS3",
  "term_label": "ubiquitin-like ligase-substrate adaptor activity",
  "gene_symbol": "KLHL28",
  "gene_name": "Kelch-like protein 28",
  "term_id": "GO:1990756"
}